{
  "gene_name": "Macrophage metalloelastase",
  "term_id": "GO:0030198",
  "term_label": "extracellular matrix organization",
  "gene_symbol": "MMP12",
  "gene": "UniProtKB:P39900"
}